{
  "gene": "UniProtKB:Q9UMX3",
  "term_label": "channel activity",
  "gene_name": "Bcl-2-related ovarian killer protein",
  "gene_symbol": "BOK",
  "term_id": "GO:0015267"
}